{
  "gene": "UniProtKB:Q14571",
  "term_id": "GO:0005886",
  "term_label": "plasma membrane",
  "gene_symbol": "ITPR2",
  "gene_name": "Inositol 1,4,5-trisphosphate receptor type 2"
}